BRCA1-C complex [GO:0070533] (cellular component) References: PMID:15485915, PMID:16391231 Sources: GOC:mah Relationships: is a type of nuclear protein-containing complex [GO:0140513] Definition: A protein complex that contains the BRCA1-BARD1 heterodimer, CtIP and Mre11/Rad50/NBS1 (M/R/N) complex, and binds to DNA at DNA damage sites. BRCA1-C binding ta damaged DNA is required for DNA damage-induced Chk1 phosphorylation and the G2/M transition checkpoint.